{
  "term_label": "canonical Wnt signaling pathway",
  "gene": "UniProtKB:Q9GZT5",
  "term_id": "GO:0060070",
  "gene_name": "Protein Wnt-10a",
  "gene_symbol": "WNT10A"
}